{
  "gene": "UniProtKB:Q9Y6D9",
  "term_id": "GO:0000776",
  "gene_name": "Mitotic spindle assembly checkpoint protein MAD1",
  "gene_symbol": "MAD1L1",
  "term_label": "kinetochore"
}